{
  "gene_name": "Ras-related protein R-Ras",
  "term_id": "GO:0007163",
  "gene": "UniProtKB:P10301",
  "gene_symbol": "RRAS",
  "term_label": "establishment or maintenance of cell polarity"
}